{
  "gene_name": "Protein lifeguard 3",
  "term_id": "GO:0005262",
  "gene": "UniProtKB:Q969X1",
  "gene_symbol": "TMBIM1",
  "term_label": "calcium channel activity"
}